{
  "gene_symbol": "OVOL3",
  "term_label": "DNA-binding transcription factor activity, RNA polymerase II-specific",
  "gene_name": "Putative transcription factor ovo-like protein 3",
  "gene": "UniProtKB:O00110",
  "term_id": "GO:0000981"
}